{
  "gene_name": "Extracellular glycoprotein lacritin",
  "term_label": "secretory granule",
  "gene_symbol": "LACRT",
  "term_id": "GO:0030141",
  "gene": "UniProtKB:Q9GZZ8"
}